{
  "gene": "UniProtKB:Q93097",
  "term_id": "GO:0005125",
  "gene_name": "Protein Wnt-2b",
  "gene_symbol": "WNT2B",
  "term_label": "cytokine activity"
}